{
  "term_id": "GO:0016887",
  "gene_name": "Kinesin-like protein KIF2C",
  "gene_symbol": "KIF2C",
  "gene": "UniProtKB:Q99661",
  "term_label": "ATP hydrolysis activity"
}